{
  "gene": "UniProtKB:Q8NI22",
  "term_label": "Unknown cellular component",
  "term_id": "UNKNOWN:0003",
  "gene_name": "Multiple coagulation factor deficiency protein 2",
  "gene_symbol": "MCFD2"
}